{
  "term_label": "G protein-coupled receptor activity",
  "gene": "UniProtKB:P41180",
  "gene_symbol": "CASR",
  "gene_name": "Extracellular calcium-sensing receptor",
  "term_id": "GO:0004930"
}